{
  "term_id": "UNKNOWN:0001",
  "gene_name": "Uncharacterized protein",
  "gene_symbol": "A0A494C0B9",
  "gene": "UniProtKB:A0A494C0B9",
  "term_label": "Unknown molecular function"
}